{
  "term_id": "GO:0010976",
  "gene": "UniProtKB:Q99578",
  "gene_name": "GTP-binding protein Rit2",
  "term_label": "positive regulation of neuron projection development",
  "gene_symbol": "RIT2"
}